{
  "gene_symbol": "VAPB",
  "term_id": "GO:0090158",
  "gene": "UniProtKB:O95292",
  "gene_name": "Vesicle-associated membrane protein-associated protein B_C",
  "term_label": "endoplasmic reticulum membrane organization"
}